{
  "gene_symbol": "TUBG2",
  "term_label": "mitotic spindle organization",
  "gene": "UniProtKB:Q9NRH3",
  "gene_name": "Tubulin gamma-2 chain",
  "term_id": "GO:0007052"
}